valyl-tRNA aminoacylation [GO:0006438] (biological process) Relationships: is a type of tRNA aminoacylation for protein translation [GO:0006418] Subtypes: cytosolic valyl-tRNA aminoacylation [GO:0061475], mitochondrial valyl-tRNA aminoacylation [GO:0070185] Definition: The process of coupling valine to valyl-tRNA, catalyzed by valyl-tRNA synthetase. The valyl-tRNA synthetase is a class-I synthetase. The activated amino acid is transferred to the 2'-OH group of a valine-accetping tRNA. The 2'-O-aminoacyl-tRNA will ultimately migrate to the 3' position via transesterification. Sources: GOC:mcc, ISBN:0716730510